formate C-acetyltransferase activity [GO:0008861] (molecular function) Also known as: PFL, formate acetyltransferase activity Sources: RHEA:11844 Definition: Catalysis of the reaction: acetyl-CoA + formate = CoA + pyruvate. Relationships: is_a C-acetyltransferase activity [GO:0016453]